{
  "gene_symbol": "KCNJ8",
  "gene_name": "ATP-sensitive inward rectifier potassium channel 8",
  "gene": "UniProtKB:Q15842",
  "term_id": "GO:0005242",
  "term_label": "inward rectifier potassium channel activity"
}